{
  "gene_name": "Signal recognition particle subunit SRP54",
  "gene": "UniProtKB:P61011",
  "gene_symbol": "SRP54",
  "term_label": "cytosol",
  "term_id": "GO:0005829"
}